{
  "gene": "UniProtKB:O60320",
  "term_id": "UNKNOWN:0001",
  "gene_name": "Protein ENTREP2",
  "gene_symbol": "ENTREP2",
  "term_label": "Unknown molecular function"
}